{
  "gene": "UniProtKB:Q8TCT8",
  "gene_symbol": "SPPL2A",
  "gene_name": "Signal peptide peptidase-like 2A",
  "term_id": "GO:0030660",
  "term_label": "Golgi-associated vesicle membrane"
}